{
  "term_label": "long-term synaptic potentiation",
  "term_id": "GO:0060291",
  "gene": "UniProtKB:Q9UI40",
  "gene_name": "Sodium_potassium_calcium exchanger 2",
  "gene_symbol": "SLC24A2"
}